{
  "gene_name": "Fibrous sheath-interacting protein 2",
  "term_id": "UNKNOWN:0002",
  "term_label": "Unknown biological process",
  "gene_symbol": "FSIP2",
  "gene": "UniProtKB:Q5CZC0"
}